anther development [GO:0048653] (biological process) Definition: The process whose specific outcome is the progression of the anther over time, from its formation to the mature structure. Sources: GOC:jid, GOC:sm Relationships: is a type of developmental process involved in reproduction [GO:0003006]; is_a anatomical structure development [GO:0048856]; is part of GO:0048443